{
  "term_id": "GO:0005925",
  "gene": "UniProtKB:Q15942",
  "gene_symbol": "ZYX",
  "term_label": "focal adhesion",
  "gene_name": "Zyxin"
}